response to hepatocyte growth factor [GO:0035728] (biological process) Subtypes: GO:0035729 Sources: GOC:bf Relationships: is a type of response to growth factor [GO:0070848] Definition: Any process that results in a change in state or activity of a cell or an organism (in terms of movement, secretion, enzyme production, gene expression, etc.) as a result of a hepatocyte growth factor stimulus. Also known as: response to HGF stimulus, response to hepatocyte growth factor stimulus